{
  "gene_name": "Geminin coiled-coil domain-containing protein 1",
  "term_id": "GO:0003712",
  "gene_symbol": "GMNC",
  "term_label": "transcription coregulator activity",
  "gene": "UniProtKB:A6NCL1"
}